{
  "gene_symbol": "C6orf163",
  "gene_name": "Uncharacterized protein C6orf163",
  "term_label": "Unknown cellular component",
  "term_id": "UNKNOWN:0003",
  "gene": "UniProtKB:Q5TEZ5"
}